{
  "term_id": "GO:0017046",
  "gene_name": "Prolactin receptor",
  "term_label": "peptide hormone binding",
  "gene_symbol": "PRLR",
  "gene": "UniProtKB:P16471"
}